mating-type a-factor pheromone receptor activity [GO:0004933] (molecular function) Also known as: class D G protein coupled receptor activity, class D G-protein coupled receptor activity, class D G-protein-coupled receptor activity, class D GPCR activity Sources: GOC:mah Relationships: is a type of mating-type factor pheromone receptor activity [GO:0004932]; is a type of peptide pheromone receptor activity [GO:0036318] Definition: Combining with the mating-type a-factor pheromone to initiate a change in cell activity.